{
  "gene_symbol": "FBXL3",
  "term_id": "GO:0005634",
  "gene_name": "F-box_LRR-repeat protein 3",
  "term_label": "nucleus",
  "gene": "UniProtKB:Q9UKT7"
}